{
  "term_id": "GO:0051321",
  "gene_symbol": "STRA8",
  "gene": "UniProtKB:Q7Z7C7",
  "gene_name": "Stimulated by retinoic acid gene 8 protein homolog",
  "term_label": "meiotic cell cycle"
}